regulation of endocardial cushion cell differentiation [GO:0120074] (biological process) Definition: Any process that modulates the frequency, rate or extent of cell differentiation, the process in which a relatively unspecialized cell acquires the specialized structural and/or functional features of an endocardial cushion cell. Subtypes: positive regulation of endocardial cushion cell differentiation [GO:0120075], GO:0120076 Sources: GOC:BHF, GOC:BHF_miRNA, GOC:rph Relationships: is a type of GO:1905207; regulates endocardial cushion cell differentiation [GO:0061443]